{
  "gene": "UniProtKB:A0PJX8",
  "term_id": "UNKNOWN:0002",
  "gene_name": "Transmembrane protein 82",
  "term_label": "Unknown biological process",
  "gene_symbol": "TMEM82"
}